nuclear cortisol receptor activity [GO:0031963] (molecular function) Relationships: is a type of nuclear glucocorticoid receptor activity [GO:0004883] Definition: A nuclear receptor activity regulated by cortisol binding and modulating the transcription of specific gene sets transcribed by RNA polymerase II. Also known as: cortisol receptor activity References: PMID:12511169 Sources: GOC:mah